purine-containing compound transmembrane transport [GO:0072530] (BP) Sources: GOC:mah Subtypes: GO:0015860, acetyl-CoA transmembrane transport [GO:0035348], coenzyme A transmembrane transport [GO:0035349], GO:0035352, GO:0071106, mitochondrial ADP transmembrane transport [GO:0140021], purine nucleotide import into lysosome [GO:0141013], 5'-adenylyl sulfate transmembrane transport [GO:1902558], 3'-phospho-5'-adenylyl sulfate transmembrane transport [GO:1902559], GO:1903790, purine nucleobase transmembrane transport [GO:1904823], mitochondrial ATP transmembrane transport [GO:1990544] Definition: The process in which a purine-containing compound is transported across a membrane. A purine-containing compound is any compound that contains purine or a formal derivative thereof. Note: Note that this term is not intended for use in annotating lateral movement within membranes. Also known as: purine-containing compound membrane transport Relationships: is a type of transmembrane transport [GO:0055085]; is a type of nitrogen compound transport [GO:0071705]